protein-RNA sequence-specific adaptor activity [GO:0160134] (MF) Relationships: is a type of protein-RNA adaptor activity [GO:0140517] References: PMID:14749727, PMID:17036044 Definition: A protein adaptor activity characterized by the capacity to selectively recognize and interact with RNA molecules in a sequence-specific manner. Entities possessing this activity typically exhibit discerning binding preferences for specific nucleotide sequences within RNA molecules, enabling the identification and engagement of distinct RNA motifs or structural elements. This function is integral to various biological processes, including RNA processing, transport, and regulatory mechanisms, contributing to the specificity and precision of cellular RNA-related activities.